{
  "term_label": "neuron differentiation",
  "gene": "UniProtKB:O60488",
  "gene_symbol": "ACSL4",
  "term_id": "GO:0030182",
  "gene_name": "Long-chain-fatty-acid--CoA ligase 4"
}